{
  "gene": "UniProtKB:Q9UL12",
  "term_id": "GO:0005759",
  "gene_symbol": "SARDH",
  "term_label": "mitochondrial matrix",
  "gene_name": "Sarcosine dehydrogenase, mitochondrial"
}